{
  "gene_name": "ADP-ribosylation factor 6",
  "term_label": "cytoplasm",
  "gene": "UniProtKB:P62330",
  "gene_symbol": "ARF6",
  "term_id": "GO:0005737"
}